abscisic acid transmembrane transporter activity [GO:0090440] (molecular function) Definition: Enables the transfer of abscisic acid from one side of a membrane to the other. Sources: GOC:tb Also known as: abscisic acid transporter activity Relationships: is a type of monocarboxylic acid transmembrane transporter activity [GO:0008028]; is_a alcohol transmembrane transporter activity [GO:0015665]; is a type of lipid transmembrane transporter activity [GO:0170055]; is part of abscisic acid transport [GO:0080168]